{
  "gene_symbol": "STX10",
  "term_label": "SNARE complex",
  "term_id": "GO:0031201",
  "gene": "UniProtKB:O60499",
  "gene_name": "Syntaxin-10"
}